rDNA binding [GO:0000182] (MF) Relationships: is a type of sequence-specific double-stranded DNA binding [GO:1990837] Subtypes: rDNA spacer replication fork barrier binding [GO:0043110], 5S rDNA binding [GO:0080084] Also known as: ribosomal DNA binding Definition: Binding to a DNA sequence encoding a ribosomal RNA. Sources: GOC:mah